{
  "gene_symbol": "CLUH",
  "term_label": "cytoplasm",
  "term_id": "GO:0005737",
  "gene": "UniProtKB:O75153",
  "gene_name": "Clustered mitochondria protein homolog"
}